{
  "gene_name": "Olfactory receptor 2B11",
  "gene_symbol": "OR2B11",
  "term_id": "GO:0050911",
  "term_label": "detection of chemical stimulus involved in sensory perception of smell",
  "gene": "UniProtKB:Q5JQS5"
}